nucleoside transmembrane transporter activity [GO:0005337] (molecular function) Definition: Enables the transfer of a nucleoside, a nucleobase linked to either beta-D-ribofuranose (ribonucleoside) or 2-deoxy-beta-D-ribofuranose, (a deoxyribonucleotide) from one side of a membrane to the other. Sources: GOC:ai Also known as: intracellular nucleoside transmembrane transporter activity Relationships: is a type of nucleobase-containing compound transmembrane transporter activity [GO:0015932]; is a type of carbohydrate derivative transmembrane transporter activity [GO:1901505]; is part of nucleoside transmembrane transport [GO:1901642] Subtypes: GO:0005415, nucleoside transmembrane transporter activity, against a concentration gradient [GO:0010174], purine nucleoside transmembrane transporter activity [GO:0015211], GO:0015214, GO:0015395, nucleoside-specific channel forming porin activity [GO:0015471], GO:0015506, nicotinamide riboside transmembrane transporter activity [GO:0034257], GO:0160286